{
  "gene_name": "Glutamine synthetase",
  "term_id": "GO:0006542",
  "gene_symbol": "GLUL",
  "gene": "UniProtKB:P15104",
  "term_label": "glutamine biosynthetic process"
}